{
  "gene_name": "Transcription factor SOX-12",
  "gene_symbol": "SOX12",
  "term_label": "positive regulation of transcription by RNA polymerase II",
  "gene": "UniProtKB:O15370",
  "term_id": "GO:0045944"
}